cytoplasm [GO:0005737] (cellular component) Relationships: is a type of cellular anatomical structure [GO:0110165]; is part of GO:0005622 Definition: The contents of a cell excluding the plasma membrane and nucleus, but including other subcellular structures. Sources: ISBN:0198547684 Subtypes: cell cortex [GO:0005938], sarcoplasm [GO:0016528], pole plasm [GO:0045495], GO:0099568, ooplasm [GO:1990917]